histone H2BS14 kinase activity [GO:0044025] (molecular function) References: PMID:15652479 Relationships: is a type of GO:0004674; is_a histone H2B kinase activity [GO:0140998] Definition: Catalysis of the reaction: histone H2B-serine (position 14) + ATP = histone H2B-phosphoserine (position 14) + ADP. This reaction is the addition of a phosphate group to the serine residue at position 14 of histone H2B. Also known as: histone kinase activity (H2B-S14 specific), histone serine kinase activity (H2B-S14 specific), histone-serine kinase activity (H2B-S14 specific) Note: Note that the residue position corresponds to the canonical human H2B histone (UniProtKB:P62807); the N-terminus of histone H2B is divergent across eukaryotes; make sure that the paper clearly references the human protein for the position of this modification to use this term. Residue 1 is the first residue following removal of the initiating Methionine (Met). Corresponds to Serine 10 in yeast (PMID:15652479). Note that each histone is encoded by multiple genes, and sequences may vary across different genes within an organism.